protein-fructosamine 3-kinase activity [GO:0102194] (molecular function) Definition: Catalysis of the reaction: ATP + a [protein]-N6-D-fructosyl-L-lysine = ADP + H+ + a [protein]-N6-(3-O-phospho-D-fructosyl)-L-lysine. References: PMID:11016445 Sources: EC:2.7.1.171, GOC:pz Also known as: fructosamine-3-kinase activity Relationships: is a type of GO:0016301; is_a catalytic activity, acting on a protein [GO:0140096]